myotube cell development [GO:0014904] (biological process) Relationships: is a type of striated muscle cell development [GO:0055002]; is part of myotube differentiation [GO:0014902] Subtypes: GO:0014906, skeletal muscle fiber development [GO:0048741] Sources: GOC:mtg_muscle Definition: The process aimed at the progression of a myotube cell over time, from initial commitment of the cell to a specific fate, to the fully functional differentiated cell. Myotubes are multinucleated cells that are formed when proliferating myoblasts exit the cell cycle, differentiate and fuse.